cellular response to freezing [GO:0071497] (biological process) Relationships: is a type of response to freezing [GO:0050826]; is a type of cellular response to cold [GO:0070417] Also known as: antifreeze activity, ice nucleation inhibitor activity Definition: Any process that results in a change in state or activity of a cell (in terms of movement, secretion, enzyme production, gene expression, etc.) as a result of a freezing stimulus, temperatures below 0 degrees Celsius. Sources: GOC:mah